cellular response to rapamycin [GO:0072752] (biological process) Definition: Any process that results in a change in state or activity of a cell (in terms of movement, secretion, enzyme production, gene expression, etc.) as a result of a rapamycin stimulus. Sources: GOC:TermGenie Relationships: is a type of cellular response to ether [GO:0071362]; is a type of cellular response to alcohol [GO:0097306]; is a type of response to rapamycin [GO:1901355]; is a type of GO:1901655; is a type of GO:1901699